{
  "gene_symbol": "HDLBP",
  "term_id": "GO:0003729",
  "gene": "UniProtKB:Q00341",
  "gene_name": "Vigilin",
  "term_label": "mRNA binding"
}